{
  "gene_name": "SWI_SNF-related matrix-associated actin-dependent regulator of chromatin subfamily B member 1",
  "gene_symbol": "SMARCB1",
  "term_label": "nBAF complex",
  "term_id": "GO:0071565",
  "gene": "UniProtKB:Q12824"
}